{
  "gene_name": "Centromere protein U",
  "term_label": "nucleus",
  "gene": "UniProtKB:Q71F23",
  "term_id": "GO:0005634",
  "gene_symbol": "CENPU"
}